{
  "term_id": "GO:0030334",
  "gene": "UniProtKB:O14604",
  "gene_name": "Thymosin beta-4, Y-chromosomal",
  "term_label": "regulation of cell migration",
  "gene_symbol": "TMSB4Y"
}